{
  "gene_symbol": "PLAC4",
  "gene_name": "Placenta-specific protein 4",
  "term_id": "UNKNOWN:0003",
  "term_label": "Unknown cellular component",
  "gene": "UniProtKB:Q8WY50"
}